nephrogenic mesenchyme development [GO:0072076] (biological process) Definition: The biological process whose specific outcome is the progression of a nephrogenic mesenchyme from an initial condition to its mature state. This process begins with the formation of nephrogenic mesenchyme and ends with the mature structure. Nephrogenic mesenchyme is the tissue made up of loosely connected mesenchymal cells in the nephron. Relationships: is a type of kidney mesenchyme development [GO:0072074]; is part of nephron development [GO:0072006] Sources: GOC:mtg_kidney_jan10